positive regulation of presynaptic cytosolic calcium concentration [GO:0099533] (biological process) Sources: GOC:dos Definition: Any process that increases the concentration of calcium ions in the presynaptic cytosol. Subtypes: induction of synaptic vesicle exocytosis by positive regulation of presynaptic cytosolic calcium ion concentration [GO:0099703] Relationships: is a type of GO:0007204; BFO_0000066 presynapse [GO:0098793]